non-collagenous component of interstitial matrix [GO:0140149] (cellular component) Definition: The non-collagenous component of interstitial extracellular matrices, including glycoprotein like fibronectin and elastin. References: PMID:21123617, PMID:25701227, PMID:33605520, PMID:39223427 Relationships: is a type of external encapsulating structure [GO:0030312]; is part of GO:0140151